{
  "gene_symbol": "LRRC8B",
  "gene": "UniProtKB:Q6P9F7",
  "gene_name": "Volume-regulated anion channel subunit LRRC8B",
  "term_label": "cytoplasm",
  "term_id": "GO:0005737"
}